{
  "gene": "UniProtKB:Q6PCT2",
  "term_id": "GO:0003712",
  "term_label": "transcription coregulator activity",
  "gene_name": "F-box_LRR-repeat protein 19",
  "gene_symbol": "FBXL19"
}